{
  "term_id": "GO:0070286",
  "term_label": "axonemal dynein complex assembly",
  "gene": "UniProtKB:Q9NQM4",
  "gene_name": "Dynein axonemal assembly factor 6",
  "gene_symbol": "DNAAF6"
}